{
  "term_id": "GO:0001755",
  "gene_name": "Semaphorin-6D",
  "gene_symbol": "SEMA6D",
  "gene": "UniProtKB:Q8NFY4",
  "term_label": "neural crest cell migration"
}